peptidyl-N-phospho-arginine dephosphorylation [GO:0098628] (BP) References: PMID:23770242 Definition: The removal of phosphate residues from peptidyl-N-phospho-arginine to form peptidyl-arginine. Relationships: is a type of protein dephosphorylation [GO:0006470]